{
  "gene_symbol": "CD244",
  "term_label": "MHC class I protein binding",
  "gene_name": "Natural killer cell receptor 2B4",
  "term_id": "GO:0042288",
  "gene": "UniProtKB:Q9BZW8"
}